{
  "gene_name": "Visual system homeobox 1",
  "gene": "UniProtKB:Q9NZR4",
  "gene_symbol": "VSX1",
  "term_label": "nucleus",
  "term_id": "GO:0005634"
}